{
  "gene_symbol": "KPNA1",
  "gene_name": "Importin subunit alpha-5",
  "term_id": "GO:0099527",
  "term_label": "postsynapse to nucleus signaling pathway",
  "gene": "UniProtKB:P52294"
}